{
  "term_id": "GO:0019532",
  "term_label": "oxalate transport",
  "gene_symbol": "SLC26A7",
  "gene": "UniProtKB:Q8TE54",
  "gene_name": "Anion exchange transporter"
}